{
  "gene_symbol": "PLEKHJ1",
  "gene_name": "Pleckstrin homology domain-containing family J member 1",
  "term_id": "GO:0055037",
  "gene": "UniProtKB:Q9NW61",
  "term_label": "recycling endosome"
}